Systematic synonym [go#systematic:synonym]